induction of conjugation upon nitrogen starvation [GO:0031142] (biological process) Definition: The process in which a cell initiates conjugation with cellular fusion upon nitrogen starvation. Sources: GOC:mah Relationships: is a type of GO:0006995; is a type of GO:0031140 Regulation: regulated by regulation of induction of conjugation upon nitrogen starvation [GO:0060905]